{
  "gene": "UniProtKB:P06133",
  "term_id": "GO:0008210",
  "gene_name": "UDP-glucuronosyltransferase 2B4",
  "gene_symbol": "UGT2B4",
  "term_label": "estrogen metabolic process"
}